long-chain fatty acid metabolic process [GO:0001676] (BP) Note: While there is not universal consensus on the lengths of short-, medium-, long- and very-long-chain fatty acids, the GO uses the definitions in ChEBI (see CHEBI:26666, CHEBI:59554, CHEBI:15904 and CHEBI:27283). Subtypes: jasmonic acid metabolic process [GO:0009694], GO:0019369, leukotriene B4 metabolic process [GO:0036102], alpha-linolenic acid metabolic process [GO:0036109], long-chain fatty acid catabolic process [GO:0042758], long-chain fatty acid biosynthetic process [GO:0042759], linoleic acid metabolic process [GO:0043651], leukotriene A4 metabolic process [GO:1901751], phytanic acid metabolic process [GO:1903512], lipoxin A4 metabolic process [GO:2001302], GO:2001304 Relationships: is a type of fatty acid metabolic process [GO:0006631] Definition: The chemical reactions and pathways involving a long-chain fatty acid. A long-chain fatty acid has an aliphatic tail containing 13 to 22 carbons. Sources: GOC:ajp Also known as: long-chain fatty acid metabolism